{
  "gene_name": "HLA class II histocompatibility antigen, DP beta 1 chain",
  "term_id": "GO:0023026",
  "gene_symbol": "HLA-DPB1",
  "gene": "UniProtKB:P04440",
  "term_label": "MHC class II protein complex binding"
}